{
  "gene_symbol": "SLC37A2",
  "gene": "UniProtKB:Q8TED4",
  "gene_name": "Glucose-6-phosphate exchanger SLC37A2",
  "term_label": "endoplasmic reticulum membrane",
  "term_id": "GO:0005789"
}